{
  "gene_symbol": "PMS2CL",
  "term_label": "Unknown biological process",
  "gene": "UniProtKB:Q68D20",
  "term_id": "UNKNOWN:0002",
  "gene_name": "Protein PMS2CL"
}